{
  "gene": "UniProtKB:P21579",
  "term_id": "GO:0070382",
  "gene_name": "Synaptotagmin-1",
  "term_label": "exocytic vesicle",
  "gene_symbol": "SYT1"
}